rejection of pollen from other species [GO:1990109] (biological process) Definition: The recognition and rejection of pollen of one species by cells in the stigma of another species. Relationships: is a type of GO:0048544; is part of pollen-pistil interaction [GO:0009875] References: PMID:21205670 Also known as: unilateral interspecific incompatibility